{
  "gene": "UniProtKB:Q9NUY8",
  "term_id": "GO:1990403",
  "gene_name": "TBC1 domain family member 23",
  "term_label": "embryonic brain development",
  "gene_symbol": "TBC1D23"
}